{
  "term_label": "Unknown biological process",
  "gene": "UniProtKB:Q3SXR2",
  "term_id": "UNKNOWN:0002",
  "gene_symbol": "C3orf36",
  "gene_name": "Uncharacterized protein C3orf36"
}